{
  "term_label": "Unknown cellular component",
  "term_id": "UNKNOWN:0003",
  "gene": "UniProtKB:Q8N961",
  "gene_symbol": "ABTB2",
  "gene_name": "Ankyrin repeat and BTB_POZ domain-containing protein 2"
}